{
  "gene": "UniProtKB:Q6VUC0",
  "term_label": "DNA-binding transcription activator activity, RNA polymerase II-specific",
  "gene_name": "Transcription factor AP-2-epsilon",
  "gene_symbol": "TFAP2E",
  "term_id": "GO:0001228"
}